{
  "term_id": "GO:0007015",
  "gene": "UniProtKB:Q9ULV0",
  "gene_name": "Unconventional myosin-Vb",
  "term_label": "actin filament organization",
  "gene_symbol": "MYO5B"
}